{
  "gene_name": "Phosphoenolpyruvate carboxykinase [GTP], mitochondrial",
  "term_label": "hepatocyte differentiation",
  "term_id": "GO:0070365",
  "gene_symbol": "PCK2",
  "gene": "UniProtKB:Q16822"
}